serine-type endopeptidase inhibitor activity [GO:0004867] (molecular function) Also known as: serine protease inhibitor activity, serine proteinase inhibitor activity, serpin activity Definition: Binds to and stops, prevents or reduces the activity of a serine-type endopeptidase. Sources: GOC:ai Relationships: is a type of endopeptidase inhibitor activity [GO:0004866]; negatively regulates serine-type endopeptidase activity [GO:0004252]